{
  "term_id": "GO:0030027",
  "term_label": "lamellipodium",
  "gene_symbol": "VIL1",
  "gene": "UniProtKB:P09327",
  "gene_name": "Villin-1"
}